{
  "gene_name": "25-hydroxyvitamin D-1 alpha hydroxylase, mitochondrial",
  "gene_symbol": "CYP27B1",
  "term_id": "GO:0036378",
  "gene": "UniProtKB:O15528",
  "term_label": "calcitriol biosynthetic process from calciol"
}